viral RNA-directed RNA polymerase complex [GO:0031381] (cellular component) References: PMID:15574411, PMID:15613301 Sources: GOC:mah Definition: A virus-specific protein complex that possesses RNA-dependent RNA polymerase activity and replicates the genome of an RNA virus. Relationships: is_a RNA-directed RNA polymerase complex [GO:0031379]